{
  "gene_name": "Solute carrier family 13 member 2",
  "gene": "UniProtKB:Q13183",
  "term_id": "GO:0015742",
  "term_label": "alpha-ketoglutarate transport",
  "gene_symbol": "SLC13A2"
}